{
  "gene_name": "N-fatty-acyl-amino acid synthase_hydrolase PM20D1",
  "term_label": "hydrolase activity, acting on carbon-nitrogen (but not peptide) bonds, in linear amides",
  "gene_symbol": "PM20D1",
  "term_id": "GO:0016811",
  "gene": "UniProtKB:Q6GTS8"
}